positive regulation of oomycete sporangium development [GO:0075323] (biological process) Definition: Any process that activates, maintains or increases the frequency, rate or extent of oomycete sporangium development, a process that leads to the formation of oomycete sporangium, a single-celled or many-celled structure that germinates directly to form an infection hypha or differentiate, through specialized cleavage vesicles, into between 10 and 30 zoospores, which is laterally flagellated. Sources: GOC:pamgo_curators Relationships: is a type of positive regulation of sporulation [GO:0043938]; is_a positive regulation of sporangium development [GO:0075311]; is a type of GO:0075322; is a type of positive regulation of asexual reproduction [GO:1903666]; positively regulates oomycete sporangium development [GO:0075321]